regulation of ecdysteroid biosynthetic process [GO:0007554] (biological process) Also known as: regulation of ecdysteroid anabolism, regulation of ecdysteroid biosynthesis, regulation of ecdysteroid formation, regulation of ecdysteroid synthesis Subtypes: GO:0045997, positive regulation of ecdysteroid biosynthetic process [GO:0045998] Relationships: is_a GO:0007553; is a type of regulation of ketone biosynthetic process [GO:0010566]; is a type of regulation of steroid hormone biosynthetic process [GO:0090030]; regulates ecdysteroid biosynthetic process [GO:0045456] Sources: GOC:go_curators Definition: Any process that modulates the frequency, rate or extent of the chemical reactions and pathways resulting in the formation of ecdysteroids.